{
  "gene_symbol": "STXBP1",
  "term_id": "GO:0099525",
  "term_label": "presynaptic dense core vesicle exocytosis",
  "gene": "UniProtKB:P61764",
  "gene_name": "Syntaxin-binding protein 1"
}